negative regulation of synaptic vesicle endocytosis [GO:1900243] (biological process) Definition: Any process that stops, prevents or reduces the frequency, rate or extent of synaptic vesicle endocytosis. Also known as: down regulation of synaptic vesicle endocytosis, down-regulation of synaptic vesicle endocytosis, downregulation of synaptic vesicle endocytosis, inhibition of synaptic vesicle endocytosis, down regulation of synaptic vesicle retrieval, down-regulation of synaptic vesicle retrieval, downregulation of synaptic vesicle retrieval, inhibition of synaptic vesicle retrieval, negative regulation of synaptic vesicle retrieval Subtypes: negative regulation of synaptic vesicle uncoating [GO:1903389] Relationships: is a type of negative regulation of endocytosis [GO:0045806]; is a type of regulation of synaptic vesicle endocytosis [GO:1900242]; is a type of negative regulation of synaptic vesicle recycling [GO:1903422]; negatively regulates synaptic vesicle endocytosis [GO:0048488] Sources: GOC:BHF, GOC:TermGenie